{
  "term_id": "GO:0005634",
  "term_label": "nucleus",
  "gene_name": "NAD-dependent protein deacetylase sirtuin-7",
  "gene_symbol": "SIRT7",
  "gene": "UniProtKB:Q9NRC8"
}